{
  "gene_symbol": "GAGE2C",
  "term_label": "Unknown biological process",
  "gene_name": "G antigen 2B_2C",
  "term_id": "UNKNOWN:0002",
  "gene": "UniProtKB:Q13066"
}